{
  "gene": "UniProtKB:A0A087WT02",
  "gene_name": "T cell receptor alpha variable 9-2",
  "gene_symbol": "TRAV9-2",
  "term_label": "immunoglobulin complex",
  "term_id": "GO:0019814"
}